{
  "gene": "UniProtKB:Q8N6C8",
  "term_id": "GO:0032396",
  "gene_name": "Leukocyte immunoglobulin-like receptor subfamily A member 3",
  "term_label": "inhibitory MHC class I receptor activity",
  "gene_symbol": "LILRA3"
}